{
  "gene_symbol": "ZFAND1",
  "gene": "UniProtKB:Q8TCF1",
  "term_id": "GO:0010494",
  "gene_name": "AN1-type zinc finger protein 1",
  "term_label": "cytoplasmic stress granule"
}